{
  "gene_symbol": "CD93",
  "term_id": "GO:0001525",
  "gene": "UniProtKB:Q9NPY3",
  "gene_name": "Complement component C1q receptor",
  "term_label": "angiogenesis"
}